F-9775A biosynthetic process [GO:1900611] (biological process) Also known as: F-9775A anabolism, F-9775A biosynthesis, F-9775A formation, F-9775A synthesis Regulation: regulated by regulation of F-9775A biosynthetic process [GO:1900670]; negatively regulated by negative regulation of F-9775A biosynthetic process [GO:1900671]; positively regulated by positive regulation of F-9775A biosynthetic process [GO:1900672] Definition: The chemical reactions and pathways resulting in the formation of F-9775A. Sources: GOC:TermGenie, GOC:di Relationships: is a type of GO:0030639; is a type of GO:0046189